{
  "gene_name": "Endogenous retrovirus group PABLB member 1 Env polyprotein",
  "gene": "UniProtKB:P60509",
  "term_id": "UNKNOWN:0002",
  "term_label": "Unknown biological process",
  "gene_symbol": "ERVPABLB-1"
}